response to prostaglandin [GO:0034694] (biological process) Subtypes: response to prostaglandin E [GO:0034695], response to prostaglandin F [GO:0034696], GO:0034697, cellular response to prostaglandin stimulus [GO:0071379], response to prostaglandin D [GO:0071798] Also known as: response to prostaglandin stimulus Sources: GOC:BHF, GOC:vk Relationships: is_a response to hormone [GO:0009725]; is a type of response to lipid [GO:0033993] Definition: Any process that results in a change in state or activity of a cell or an organism (in terms of movement, secretion, enzyme production, gene expression, etc.) as a result of a prostagladin stimulus.